{
  "term_label": "mitochondrial matrix",
  "term_id": "GO:0005759",
  "gene_name": "Iron-sulfur cluster assembly enzyme ISCU",
  "gene_symbol": "ISCU",
  "gene": "UniProtKB:Q9H1K1"
}